regulation of translational initiation by iron [GO:0006447] (biological process) Definition: Any process that modulates the frequency, rate or extent of the translation of certain mRNAs involved in iron metabolism; regulated by the concentration of iron. Sources: GOC:jl Subtypes: negative regulation of translational initiation by iron [GO:0045993], positive regulation of translational initiation by iron [GO:0045994] Relationships: is a type of regulation of translational initiation [GO:0006446]